{
  "gene": "UniProtKB:Q8N328",
  "term_label": "sequence-specific DNA binding",
  "term_id": "GO:0043565",
  "gene_name": "PiggyBac transposable element-derived protein 3",
  "gene_symbol": "PGBD3"
}